{
  "gene_symbol": "HEATR1",
  "term_label": "positive regulation of transcription by RNA polymerase I",
  "gene": "UniProtKB:Q9H583",
  "gene_name": "HEAT repeat-containing protein 1",
  "term_id": "GO:0045943"
}